{
  "gene_symbol": "GOLGA8O",
  "term_id": "UNKNOWN:0001",
  "gene": "UniProtKB:A6NCC3",
  "term_label": "Unknown molecular function",
  "gene_name": "Golgin subfamily A member 8O"
}